D-xylose:proton symporter activity [GO:0015519] (MF) Relationships: is a type of carbohydrate:proton symporter activity [GO:0005351]; is a type of D-xylose transmembrane transporter activity [GO:0015148] Also known as: D-xylose:hydrogen symporter activity Definition: Enables the transfer of a solute or solutes from one side of a membrane to the other according to the reaction: D-xylose(out) + H+(out) = D-xylose(in) + H+(in). Sources: TC:2.A.1.1.3